{
  "gene": "UniProtKB:A6NGG8",
  "gene_symbol": "PCARE",
  "gene_name": "Photoreceptor cilium actin regulator",
  "term_label": "protein localization to photoreceptor outer segment",
  "term_id": "GO:1903546"
}